nucleoside triphosphate diphosphatase activity [GO:0047429] (molecular function) Sources: EC:3.6.1.9 Also known as: nucleoside-triphosphate diphosphatase activity, nucleoside-triphosphate diphosphohydrolase activity, nucleoside-triphosphate pyrophosphatase activity Relationships: is a type of pyrophosphatase activity [GO:0016462] Subtypes: dUTP diphosphatase activity [GO:0004170], 8-oxo-7,8-dihydroguanosine triphosphate pyrophosphatase activity [GO:0008413], dATP diphosphatase activity [GO:0008828], 8-oxo-7,8-dihydrodeoxyguanosine triphosphate pyrophosphatase activity [GO:0035539], dITP diphosphatase activity [GO:0035870], GO:0036217, dTTP diphosphatase activity [GO:0036218], GTP diphosphatase activity [GO:0036219], ITP diphosphatase activity [GO:0036220], UTP diphosphatase activity [GO:0036221], XTP diphosphatase activity [GO:0036222], ATP diphosphatase activity [GO:0047693], dCTP diphosphatase activity [GO:0047840], 2-hydroxy-ATP hydrolase activity [GO:0106377], GO:0106378, 8-oxo-(d)RTP hydrolase activity [GO:0106379] Definition: Catalysis of the reaction: a nucleoside triphosphate + H2O = a nucleotide + H+ + diphosphate.